{
  "term_id": "GO:0030154",
  "term_label": "cell differentiation",
  "gene": "UniProtKB:Q9NX45",
  "gene_name": "Spermatogenesis- and oogenesis-specific basic helix-loop-helix-containing protein 2",
  "gene_symbol": "SOHLH2"
}